{
  "gene_symbol": "WNT16",
  "gene_name": "Protein Wnt-16",
  "term_label": "frizzled binding",
  "term_id": "GO:0005109",
  "gene": "UniProtKB:Q9UBV4"
}